{
  "gene_symbol": "A0A6Q8PFQ6",
  "gene_name": "Uncharacterized protein",
  "term_id": "UNKNOWN:0002",
  "gene": "UniProtKB:A0A6Q8PFQ6",
  "term_label": "Unknown biological process"
}